germline stem cell symmetric division [GO:0098729] (biological process) Relationships: is a type of germ-line stem cell division [GO:0042078]; is a type of symmetric stem cell division [GO:0098724] Subtypes: female germline stem cell symmetric division [GO:0062102], male germline stem cell symmetric division [GO:0098730] References: PMID:19948499 Sources: GOC:dos Definition: Division of a germline stem cell to produce two germline stem cells of the same type as the parent.